positive regulation of DNA topoisomerase (ATP-hydrolyzing) activity [GO:2000373] (biological process) Also known as: positive regulation of DNA topoisomerase IV activity, positive regulation of DNA topoisomerase type II activity, positive regulation of deoxyribonucleic topoisomerase activity, positive regulation of topoisomerase II, positive regulation of type II DNA topoisomerase activity, positive regulation of DNA topoisomerase (ATP-hydrolysing), positive regulation of DNA topoisomerase II, positive regulation of deoxyribonucleate topoisomerase, positive regulation of topoisomerase Sources: GOC:mah Relationships: is a type of positive regulation of ATP-dependent activity [GO:0032781]; is_a positive regulation of catalytic activity [GO:0043085]; positively regulates DNA topoisomerase type II (double strand cut, ATP-hydrolyzing) activity [GO:0003918] Definition: Any process that activates or increases the frequency, rate or extent of DNA topoisomerase (ATP-hydrolyzing) activity.